cell wall organization [GO:0071555] (biological process) Relationships: is a type of GO:0045229; is a type of cell wall organization or biogenesis [GO:0071554] Definition: A process that results in the assembly, arrangement of constituent parts, or disassembly of the cell wall, the rigid or semi-rigid envelope lying outside the cell membrane of plant, fungal and most prokaryotic cells, maintaining their shape and protecting them from osmotic lysis. Subtypes: plant-type cell wall organization [GO:0009664], peptidoglycan-based cell wall organization [GO:0031504], fungal-type cell wall organization [GO:0031505], GO:0042545, GO:0044277, GO:0070726, cell wall organization involved in conjugation with cellular fusion [GO:0070871], cell wall repair [GO:0071433] Also known as: cell wall organisation, cell wall organisation in other organism, cell wall organization at cellular level, cell wall organization in other organism, cellular cell wall organisation, cellular cell wall organization, cell wall organization and biogenesis Sources: GOC:mah